{
  "term_id": "GO:0009897",
  "term_label": "external side of plasma membrane",
  "gene": "UniProtKB:Q95460",
  "gene_name": "Major histocompatibility complex class I-related gene protein",
  "gene_symbol": "MR1"
}